{
  "gene_name": "Endoglin",
  "term_id": "GO:0009986",
  "gene": "UniProtKB:P17813",
  "term_label": "cell surface",
  "gene_symbol": "ENG"
}